{
  "term_label": "cellular response to hypoxia",
  "gene": "UniProtKB:Q96KS0",
  "term_id": "GO:0071456",
  "gene_symbol": "EGLN2",
  "gene_name": "Prolyl hydroxylase EGLN2"
}